{
  "gene_name": "Endoplasmin",
  "gene_symbol": "HSP90B1",
  "term_id": "GO:0006457",
  "term_label": "protein folding",
  "gene": "UniProtKB:P14625"
}